{
  "gene": "UniProtKB:Q96LA5",
  "term_label": "transmembrane signaling receptor activity",
  "gene_name": "Fc receptor-like protein 2",
  "gene_symbol": "FCRL2",
  "term_id": "GO:0004888"
}